{
  "gene_symbol": "IGKV2D-28",
  "gene": "UniProtKB:P01615",
  "term_label": "immunoglobulin complex",
  "gene_name": "Immunoglobulin kappa variable 2D-28",
  "term_id": "GO:0019814"
}